regulation of antigen processing and presentation [GO:0002577] (biological process) Definition: Any process that modulates the frequency, rate, or extent of antigen processing and presentation. Subtypes: negative regulation of antigen processing and presentation [GO:0002578], GO:0002579, regulation of antigen processing and presentation of peptide or polysaccharide antigen via MHC class II [GO:0002580], regulation of antigen processing and presentation of peptide antigen [GO:0002583], regulation of antigen processing and presentation via MHC class Ib [GO:0002592], regulation of dendritic cell antigen processing and presentation [GO:0002604], GO:0002613, regulation of macrophage antigen processing and presentation [GO:0002616], GO:0002619, regulation of B cell antigen processing and presentation [GO:0002622], regulation of T cell antigen processing and presentation [GO:0002625] Sources: GOC:add Relationships: is a type of regulation of immune system process [GO:0002682]; regulates antigen processing and presentation [GO:0019882]